{
  "gene": "UniProtKB:Q96HR9",
  "term_id": "UNKNOWN:0002",
  "gene_symbol": "REEP6",
  "term_label": "Unknown biological process",
  "gene_name": "Receptor expression-enhancing protein 6"
}